epididymosome [GO:0098875] (cellular component) Definition: A microvesicle of the epididymal fluid, from which spermatozoa acquire membrane proteins. Relationships: is a type of microvesicle [GO:1990742] References: PMID:23177142, PMID:26112475 Sources: GOC:dos, GOC:mg